protein tyrosine kinase collagen receptor activity [GO:0038062] (molecular function) Also known as: collagen RTK activity, discoidin domain receptor Relationships: is a type of transmembrane receptor protein tyrosine kinase activity [GO:0004714]; is a type of collagen receptor activity [GO:0038064]; is part of collagen-activated tyrosine kinase receptor signaling pathway [GO:0038063] References: PMID:16626936, PMID:21568710 Sources: GOC:bf, GOC:uh Definition: Combining with collagen and transmitting the signal from one side of the membrane to the other to initiate a change in cell activity by catalysis of the reaction: ATP + a protein-L-tyrosine = ADP + a protein-L-tyrosine phosphate.